diamine transaminase activity [GO:0019161] (molecular function) Definition: Catalysis of the reaction: an alpha,omega-diamine + 2-oxoglutarate = an omega-aminoaldehyde + L-glutamate. Sources: EC:2.6.1.29 Relationships: is a type of GO:0008483 Also known as: diamine aminotransferase activity, amine transaminase activity, amine-ketoacid transaminase activity, diamine-ketoglutaric transaminase activity, diamine:2-oxoglutarate aminotransferase activity